CENP-A containing chromatin assembly [GO:0034080] (biological process) Definition: The formation of chromatin containing the histone H3 variant CENP-A to form centromeric chromatin. This specialised chromatin occurs at centromeric region in point centromeres, and the central core in modular centromeres. References: PMID:18158900, PMID:19217403, PMID:35422390 Sources: GOC:mah, GOC:vw Also known as: CENP-A containing nucleosome assembly at centromere, DNA replication-independent nucleosome assembly at centromere, centromere-specific histone exchange, centromeric DNA replication-independent nucleosome assembly, CENP-A containing chromatin organization, CENP-A containing nucleosome assembly, CENP-A deposition, CENP-A loading, CenH3-containing nucleosome assembly at centromere, centromere specific nucleosome exchange, centromeric chromatin organization Relationships: is a type of GO:0006325; is part of kinetochore assembly [GO:0051382]; BFO_0000051 protein localization to CENP-A containing chromatin [GO:0061644]